{
  "gene": "UniProtKB:P22309",
  "gene_name": "UDP-glucuronosyltransferase 1A1",
  "gene_symbol": "UGT1A1",
  "term_label": "endoplasmic reticulum",
  "term_id": "GO:0005783"
}